{
  "term_id": "UNKNOWN:0003",
  "gene": "UniProtKB:Q9BQN1",
  "gene_symbol": "FAM83C",
  "gene_name": "Protein FAM83C",
  "term_label": "Unknown cellular component"
}